anterior visceral endoderm cell migration [GO:1905070] (biological process) Definition: The orderly movement of an anterior visceral endoderm cell from one site to another. References: PMID:17078044 Sources: GOC:TermGenie, GO_REF:0000091 Relationships: is a type of cell migration [GO:0016477]